{
  "gene_symbol": "ACTN3",
  "term_id": "GO:0051015",
  "gene_name": "Alpha-actinin-3",
  "gene": "UniProtKB:Q08043",
  "term_label": "actin filament binding"
}